{
  "gene_name": "C-X-C motif chemokine 5",
  "gene": "UniProtKB:P42830",
  "gene_symbol": "CXCL5",
  "term_label": "neutrophil chemotaxis",
  "term_id": "GO:0030593"
}